{
  "gene": "UniProtKB:P61077",
  "term_label": "nucleus",
  "gene_name": "Ubiquitin-conjugating enzyme E2 D3",
  "gene_symbol": "UBE2D3",
  "term_id": "GO:0005634"
}